glial cell fate determination [GO:0007403] (BP) Relationships: is a type of cell fate determination [GO:0001709]; is part of GO:0021781 Sources: GOC:go_curators, GOC:mtg_sensu Definition: The cell fate determination process in which a cell becomes capable of differentiating autonomously into a glial cell regardless of its environment; upon determination, the cell fate cannot be reversed.